mitochondrial intermembrane space [GO:0005758] (cellular component) Definition: The region between the inner and outer lipid bilayers of the mitochondrial envelope. Sources: GOC:mah Also known as: mitochondrial envelope lumen, mitochondrial membrane lumen Relationships: is a type of organelle envelope lumen [GO:0031970]; is part of mitochondrial envelope [GO:0005740]